trehalose transport in response to water deprivation [GO:0072514] (biological process) Sources: GOC:mah Relationships: is a type of trehalose transport [GO:0015771]; is part of cellular response to water deprivation [GO:0042631] Definition: The directed movement of trehalose into, out of or within a cell, or between cells, by means of some agent such as a transporter or pore, that occurs as a result of deprivation of water. Subtypes: trehalose transport in response to desiccation [GO:0072515]